{
  "gene_symbol": "EPAS1",
  "gene": "UniProtKB:Q99814",
  "term_id": "GO:0000981",
  "term_label": "DNA-binding transcription factor activity, RNA polymerase II-specific",
  "gene_name": "Endothelial PAS domain-containing protein 1"
}